{
  "term_id": "GO:0034220",
  "term_label": "monoatomic ion transmembrane transport",
  "gene": "UniProtKB:Q15825",
  "gene_name": "Neuronal acetylcholine receptor subunit alpha-6",
  "gene_symbol": "CHRNA6"
}